{
  "gene_symbol": "STX18",
  "term_id": "GO:0006890",
  "gene": "UniProtKB:Q9P2W9",
  "term_label": "retrograde vesicle-mediated transport, Golgi to endoplasmic reticulum",
  "gene_name": "Syntaxin-18"
}